{
  "gene_symbol": "PCP4L1",
  "term_label": "Unknown cellular component",
  "term_id": "UNKNOWN:0003",
  "gene": "UniProtKB:A6NKN8",
  "gene_name": "Purkinje cell protein 4-like protein 1"
}